{
  "gene_name": "Small proline-rich protein 4",
  "gene": "UniProtKB:Q96PI1",
  "term_id": "UNKNOWN:0003",
  "gene_symbol": "SPRR4",
  "term_label": "Unknown cellular component"
}